{
  "term_id": "GO:0030017",
  "gene": "UniProtKB:Q8WXH0",
  "term_label": "sarcomere",
  "gene_symbol": "SYNE2",
  "gene_name": "Nesprin-2"
}